{
  "gene": "UniProtKB:P32970",
  "gene_name": "CD70 antigen",
  "term_label": "Unknown molecular function",
  "gene_symbol": "CD70",
  "term_id": "UNKNOWN:0001"
}